{
  "gene_symbol": "RNPS1",
  "term_label": "nucleoplasm",
  "gene_name": "RNA-binding protein with serine-rich domain 1",
  "gene": "UniProtKB:Q15287",
  "term_id": "GO:0005654"
}